{
  "term_id": "GO:0043161",
  "gene_name": "Kelch-like protein 21",
  "gene": "UniProtKB:Q9UJP4",
  "gene_symbol": "KLHL21",
  "term_label": "proteasome-mediated ubiquitin-dependent protein catabolic process"
}